polyphosphate:AMP phosphotransferase activity [GO:0043751] (molecular function) References: PMID:11237733 Definition: Catalysis of the reaction: (polyphosphate)n + AMP = (polyphosphate)n-1 + ADP. Relationships: is a type of phosphotransferase activity, phosphate group as acceptor [GO:0016776] Also known as: PPT, PAP